omegasome [GO:1990462] (cellular component) Definition: Omega-shaped (as in the Greek capital letter) intracellular membrane-bounded organelle enriched in phosphatidylinositol 3-phosphate and dynamically connected to the endoplasmic reticulum. Omegasomes are the first step of the formation of autophagosomes via the phagophore assembly sites. Relationships: is a type of intracellular membrane-bounded organelle [GO:0043231]; is part of endomembrane system [GO:0012505] References: PMID:18725538, PMID:24591649 Sources: GOC:autophagy, GOC:mf